endothelial cell fate determination [GO:0060848] (biological process) Sources: GOC:dph, GOC:sdb_2009, GOC:tb Relationships: is a type of cell fate determination [GO:0001709]; is part of endothelial cell fate commitment [GO:0060839] Definition: A process involved in cell fate commitment of an endothelial cell. Once determination has taken place, a cell becomes committed to differentiate down a particular pathway regardless of its environment.